{
  "term_label": "metalloendopeptidase inhibitor activity",
  "term_id": "GO:0008191",
  "gene_name": "Testican-2",
  "gene": "UniProtKB:Q92563",
  "gene_symbol": "SPOCK2"
}